{
  "gene_name": "Ankyrin-2",
  "term_id": "GO:0043005",
  "gene": "UniProtKB:Q01484",
  "term_label": "neuron projection",
  "gene_symbol": "ANK2"
}